{
  "term_id": "UNKNOWN:0002",
  "term_label": "Unknown biological process",
  "gene_symbol": "FARP1",
  "gene": "UniProtKB:Q9Y4F1",
  "gene_name": "FERM, ARHGEF and pleckstrin domain-containing protein 1"
}